regulation of excretion [GO:0044062] (biological process) Definition: Any process that modulates the frequency, rate, or extent of excretion, the elimination by an organism of the waste products that arise as a result of metabolic activity. Sources: GOC:jl Relationships: is a type of regulation of system process [GO:0044057]; is a type of regulation of secretion [GO:0051046]; regulates excretion [GO:0007588] Subtypes: regulation of renal sodium excretion [GO:0035813], regulation of renal phosphate excretion [GO:1903402], regulation of smooth muscle contraction involved in micturition [GO:1904318], regulation of defecation [GO:2000292]